{
  "gene_symbol": "ARPC1A",
  "gene": "UniProtKB:Q92747",
  "term_label": "Arp2/3 complex-mediated actin nucleation",
  "term_id": "GO:0034314",
  "gene_name": "Actin-related protein 2_3 complex subunit 1A"
}